negative regulation of muscle cell differentiation [GO:0051148] (BP) Definition: Any process that stops, prevents, or reduces the frequency, rate or extent of muscle cell differentiation. Subtypes: negative regulation of smooth muscle cell differentiation [GO:0051151], negative regulation of striated muscle cell differentiation [GO:0051154] Relationships: is a type of negative regulation of cell differentiation [GO:0045596]; is a type of regulation of muscle cell differentiation [GO:0051147]; negatively regulates muscle cell differentiation [GO:0042692] Also known as: down regulation of muscle cell differentiation, down-regulation of muscle cell differentiation, downregulation of muscle cell differentiation, inhibition of muscle cell differentiation Sources: CL:0000187, GOC:ai